{
  "term_label": "Unknown cellular component",
  "term_id": "UNKNOWN:0003",
  "gene_symbol": "GPR171",
  "gene_name": "G-protein coupled receptor 171",
  "gene": "UniProtKB:O14626"
}